{
  "term_label": "cell-cell adhesion",
  "term_id": "GO:0098609",
  "gene": "UniProtKB:Q8IZU9",
  "gene_name": "Kin of IRRE-like protein 3",
  "gene_symbol": "KIRREL3"
}